response to host osmotic environment [GO:0075000] (biological process) Sources: GOC:pamgo_curators Also known as: response of symbiont to host osmotic environment Relationships: is a type of GO:0075136 Definition: Any process that results in a change in state or activity of the symbiont or its cell (in terms of movement, secretion, enzyme production, gene expression, etc.) as a result of the osmotic conditions in or around its host organism. The host is defined as the larger of the organisms involved in a symbiotic interaction.